{
  "term_label": "synaptic vesicle",
  "gene": "UniProtKB:Q92930",
  "term_id": "GO:0008021",
  "gene_name": "Ras-related protein Rab-8B",
  "gene_symbol": "RAB8B"
}